miltiradiene biosynthetic process [GO:1901946] (biological process) Definition: The chemical reactions and pathways resulting in the formation of miltiradiene. References: PMID:22027823 Sources: GOC:TermGenie Also known as: miltiradiene anabolism, miltiradiene biosynthesis, miltiradiene formation, miltiradiene synthesis Relationships: is a type of terpene biosynthetic process [GO:0046246]